{
  "term_label": "sterol binding",
  "term_id": "GO:0032934",
  "gene": "UniProtKB:Q9BXB4",
  "gene_name": "Oxysterol-binding protein-related protein 11",
  "gene_symbol": "OSBPL11"
}